{
  "gene_name": "Brain-specific angiogenesis inhibitor 1-associated protein 2-like protein 2",
  "gene_symbol": "BAIAP2L2",
  "gene": "UniProtKB:Q6UXY1",
  "term_label": "cytosol",
  "term_id": "GO:0005829"
}